thiamine transmembrane transport [GO:0071934] (biological process) Subtypes: GO:0030974, GO:0140125 Also known as: thiamin transmembrane transport, thiamine membrane transport, vitamin B1 transmembrane transport Relationships: is_a thiamine transport [GO:0015888]; is a type of GO:0035461; is a type of GO:0045117; is a type of GO:0072531 Sources: GOC:mah Definition: The process in which thiamine is transported across a membrane. Thiamine is vitamin B1, a water soluble vitamin present in fresh vegetables and meats, especially liver. Note: Note that this term is not intended for use in annotating lateral movement within membranes.